{
  "gene_symbol": "GKAP1",
  "term_label": "Unknown molecular function",
  "term_id": "UNKNOWN:0001",
  "gene": "UniProtKB:Q5VSY0",
  "gene_name": "G kinase-anchoring protein 1"
}